{
  "gene_symbol": "CDH2",
  "gene": "UniProtKB:P19022",
  "term_label": "apical part of cell",
  "term_id": "GO:0045177",
  "gene_name": "Cadherin-2"
}